{
  "gene_name": "Adipolin",
  "term_id": "GO:0046628",
  "term_label": "positive regulation of insulin receptor signaling pathway",
  "gene_symbol": "C1QTNF12",
  "gene": "UniProtKB:Q5T7M4"
}